{
  "gene_name": "Actin-binding protein IPP",
  "term_id": "GO:0031463",
  "term_label": "Cul3-RING ubiquitin ligase complex",
  "gene_symbol": "IPP",
  "gene": "UniProtKB:Q9Y573"
}